{
  "gene": "UniProtKB:Q9UPY6",
  "term_id": "GO:0030027",
  "gene_name": "Actin-binding protein WASF3",
  "term_label": "lamellipodium",
  "gene_symbol": "WASF3"
}